tRNA aminoacylation for nonribosomal peptide biosynthetic process [GO:0043040] (biological process) Also known as: tRNA aminoacylation for nonribosomal peptide anabolism, tRNA aminoacylation for nonribosomal peptide biosynthesis, tRNA aminoacylation for nonribosomal peptide formation, tRNA aminoacylation for nonribosomal peptide synthesis Relationships: is a type of tRNA aminoacylation [GO:0043039]; is a type of amino acid activation for nonribosomal peptide biosynthetic process [GO:0043041] Definition: The synthesis of aminoacyl tRNA by the formation of an ester bond between the 3'-hydroxyl group of the most 3' adenosine of the tRNA, to be used in nonribosomal peptide synthesis. Sources: GOC:jl